{
  "term_label": "cortical actin cytoskeleton organization",
  "term_id": "GO:0030866",
  "gene": "UniProtKB:Q6P1M3",
  "gene_symbol": "LLGL2",
  "gene_name": "LLGL scribble cell polarity complex component 2"
}